filamentous growth MAPK cascade [GO:0062031] (biological process) Definition: A MAPK cascade containing at least the Kss1 MAP kinase. It starts with the activation of Ste20, a MAP4K, which activates Ste11, a MAP3K, which in turn activate Ste7, a MAP2K, which activates Kss1. The kinases in each tier phosphorylate and activate the kinases in the downstream tier. The filamentous growth MAPK cascade is activated as a result of partial nutrient deprivation and  results in filamentous growth. References: PMID:17604854, PMID:33335117, PMID:38187743 Relationships: is a type of GO:0051403